{
  "gene_name": "Heat shock 70 kDa protein 14",
  "term_id": "GO:0044183",
  "gene": "UniProtKB:Q0VDF9",
  "term_label": "protein folding chaperone",
  "gene_symbol": "HSPA14"
}